lipopolysaccharide glucosyltransferase II activity [GO:0047270] (molecular function) Definition: Catalysis of the reaction: UDP-glucose + lipopolysaccharide = UDP + alpha-D-glucosyl-lipopolysaccharide. Also known as: LPS glucosyltransferase II activity, UDP-glucose:galactosyl-lipopolysaccharide alpha-D-glucosyltransferase activity, UDPglucose:galactosyl-lipopolysaccharide alpha-D-glucosyltransferase activity, uridine diphosphoglucose-galactosylpolysaccharide glucosyltransferase activity Sources: EC:2.4.1.73 Relationships: is a type of UDP-glucosyltransferase activity [GO:0035251]; is part of lipopolysaccharide biosynthetic process [GO:0009103]